{
  "gene_name": "Zinc finger MYM-type protein 5",
  "gene": "UniProtKB:Q9UJ78",
  "gene_symbol": "ZMYM5",
  "term_id": "UNKNOWN:0003",
  "term_label": "Unknown cellular component"
}